{
  "term_id": "UNKNOWN:0001",
  "gene": "UniProtKB:Q9H299",
  "term_label": "Unknown molecular function",
  "gene_symbol": "SH3BGRL3",
  "gene_name": "SH3 domain-binding glutamic acid-rich-like protein 3"
}